regulation of cardiac muscle cell proliferation [GO:0060043] (biological process) Also known as: regulation of heart muscle cell proliferation, regulation of cardiomyocyte proliferation Subtypes: negative regulation of cardiac muscle cell proliferation [GO:0060044], positive regulation of cardiac muscle cell proliferation [GO:0060045] Relationships: is_a regulation of cell population proliferation [GO:0042127]; is a type of regulation of cardiac muscle tissue growth [GO:0055021]; regulates GO:0060038 Sources: GOC:dph, GOC:rph Definition: Any process that modulates the frequency, rate or extent of cardiac muscle cell proliferation.